{
  "gene_symbol": "STAB1",
  "gene": "UniProtKB:Q9NY15",
  "term_label": "Unknown biological process",
  "term_id": "UNKNOWN:0002",
  "gene_name": "Stabilin-1"
}